{
  "term_id": "GO:0005794",
  "gene_symbol": "CERT1",
  "gene_name": "Ceramide transfer protein",
  "term_label": "Golgi apparatus",
  "gene": "UniProtKB:Q9Y5P4"
}